{
  "gene": "UniProtKB:P23458",
  "term_label": "cytosol",
  "term_id": "GO:0005829",
  "gene_name": "Tyrosine-protein kinase JAK1",
  "gene_symbol": "JAK1"
}